{
  "term_id": "GO:0016757",
  "gene_name": "Alpha-1,3-galactosyltransferase 2",
  "gene_symbol": "A3GALT2",
  "term_label": "glycosyltransferase activity",
  "gene": "UniProtKB:U3KPV4"
}